{
  "term_id": "GO:0048268",
  "gene": "UniProtKB:Q9NYX4",
  "gene_name": "Neuron-specific vesicular protein calcyon",
  "term_label": "clathrin coat assembly",
  "gene_symbol": "CALY"
}